{
  "term_id": "UNKNOWN:0003",
  "gene": "UniProtKB:Q9P2S6",
  "gene_name": "Ankyrin repeat and MYND domain-containing protein 1",
  "gene_symbol": "ANKMY1",
  "term_label": "Unknown cellular component"
}